{
  "term_id": "GO:0005737",
  "gene_name": "E3 ubiquitin-protein ligase SMURF1",
  "gene": "UniProtKB:Q9HCE7",
  "gene_symbol": "SMURF1",
  "term_label": "cytoplasm"
}